purine ribonucleoside triphosphate metabolic process [GO:0009205] (biological process) Definition: The chemical reactions and pathways involving purine ribonucleoside triphosphate, a compound consisting of a purine base linked to a ribose sugar esterified with triphosphate on the sugar. Sources: GOC:go_curators, ISBN:0198506732 Also known as: purine ribonucleoside triphosphate metabolism Relationships: is a type of GO:0009144 Subtypes: purine ribonucleoside triphosphate biosynthetic process [GO:0009206], GO:0009207, ATP metabolic process [GO:0046034], GTP metabolic process [GO:0046039], GO:0046041